{
  "gene_name": "Homeobox protein Nkx-6.3",
  "term_label": "DNA-binding transcription factor activity, RNA polymerase II-specific",
  "gene": "UniProtKB:A6NJ46",
  "term_id": "GO:0000981",
  "gene_symbol": "NKX6-3"
}